Sec62/Sec63 complex [GO:0031207] (cellular component) Definition: A protein complex involved in the posttranslational targeting of proteins to the ER. In yeast, it is a tetrameric complex consisting of Sec62p, Sec63p, Sec71p and Sec72p. Relationships: is a type of membrane protein complex [GO:0098796]; is a type of endoplasmic reticulum protein-containing complex [GO:0140534]; is part of GO:0031205 Also known as: ER protein translocation subcomplex, Sec62/63 complex References: PMID:12518317, PMID:14617809